{
  "gene": "UniProtKB:Q9Y2Y9",
  "gene_name": "Krueppel-like factor 13",
  "term_id": "GO:0006357",
  "gene_symbol": "KLF13",
  "term_label": "regulation of transcription by RNA polymerase II"
}